{
  "gene_name": "Transforming acidic coiled-coil-containing protein 2",
  "term_label": "cytosol",
  "gene": "UniProtKB:O95359",
  "term_id": "GO:0005829",
  "gene_symbol": "TACC2"
}